{
  "gene_symbol": "GANC",
  "term_label": "alpha-1,4-glucosidase activity",
  "gene_name": "Neutral alpha-glucosidase C",
  "term_id": "GO:0004558",
  "gene": "UniProtKB:Q8TET4"
}